{
  "term_id": "GO:0005739",
  "gene": "UniProtKB:Q8N3J5",
  "term_label": "mitochondrion",
  "gene_symbol": "PPM1K",
  "gene_name": "Protein phosphatase 1K, mitochondrial"
}